{
  "term_label": "Unknown biological process",
  "gene": "UniProtKB:O95084",
  "gene_name": "Serine protease 23",
  "term_id": "UNKNOWN:0002",
  "gene_symbol": "PRSS23"
}